{
  "gene": "UniProtKB:Q15649",
  "gene_name": "Zinc finger HIT domain-containing protein 3",
  "term_label": "pre-snoRNP complex",
  "gene_symbol": "ZNHIT3",
  "term_id": "GO:0070761"
}